{
  "gene_symbol": "MAPK13",
  "gene_name": "Mitogen-activated protein kinase 13",
  "term_label": "cytoplasm",
  "term_id": "GO:0005737",
  "gene": "UniProtKB:O15264"
}